olfactory bulb interneuron development [GO:0021891] (biological process) Definition: The process whose specific outcome is the progression of an interneuron residing in the olfactory bulb, from its initial commitment, to the fully functional differentiated cell. References: PMID:12626695 Sources: GOC:cls, GOC:dgh, GOC:dph, GOC:jid, GO_REF:0000021 Relationships: is a type of forebrain neuron development [GO:0021884]; BFO_0000050 olfactory bulb interneuron differentiation [GO:0021889]